{
  "gene_name": "Gamma-interferon-inducible lysosomal thiol reductase",
  "gene": "UniProtKB:P13284",
  "term_label": "Unknown biological process",
  "gene_symbol": "IFI30",
  "term_id": "UNKNOWN:0002"
}